{
  "gene_symbol": "U2SURP",
  "gene": "UniProtKB:O15042",
  "gene_name": "U2 snRNP-associated SURP motif-containing protein",
  "term_label": "Unknown biological process",
  "term_id": "UNKNOWN:0002"
}